{
  "gene_symbol": "SPRY4",
  "gene_name": "Protein sprouty homolog 4",
  "gene": "UniProtKB:Q9C004",
  "term_label": "negative regulation of ERK1 and ERK2 cascade",
  "term_id": "GO:0070373"
}